retinal ganglion cell axon guidance [GO:0031290] (biological process) Definition: The process in which the migration of an axon growth cone of a retinal ganglion cell (RGC) is directed to its target in the brain in response to a combination of attractive and repulsive cues. Also known as: retinal ganglion cell axon pathfinding Sources: GOC:ejs Relationships: is a type of axon guidance [GO:0007411] Regulation: regulated by regulation of retinal ganglion cell axon guidance [GO:0090259]; negatively regulated by negative regulation of retinal ganglion cell axon guidance [GO:0090260]; positively regulated by GO:1902336